{
  "term_id": "UNKNOWN:0002",
  "term_label": "Unknown biological process",
  "gene_name": "Putative uncharacterized protein LINC02902",
  "gene_symbol": "LINC02902",
  "gene": "UniProtKB:Q6ZTY9"
}